{
  "term_label": "clathrin complex",
  "gene_name": "Clathrin heavy chain 2",
  "term_id": "GO:0071439",
  "gene": "UniProtKB:P53675",
  "gene_symbol": "CLTCL1"
}